{
  "gene_symbol": "BLOC1S2",
  "gene": "UniProtKB:Q6QNY1",
  "gene_name": "Biogenesis of lysosome-related organelles complex 1 subunit 2",
  "term_id": "GO:0000930",
  "term_label": "gamma-tubulin complex"
}